negative regulation of myeloid dendritic cell antigen processing and presentation [GO:0002608] (biological process) Definition: Any process that stops, prevents, or reduces the frequency, rate, or extent of myeloid dendritic cell antigen processing and presentation. Relationships: is a type of negative regulation of dendritic cell antigen processing and presentation [GO:0002605]; is_a GO:0002607; negatively regulates myeloid dendritic cell antigen processing and presentation [GO:0002469] Sources: GOC:add Also known as: down regulation of myeloid dendritic cell antigen processing and presentation, down-regulation of myeloid dendritic cell antigen processing and presentation, downregulation of myeloid dendritic cell antigen processing and presentation, inhibition of myeloid dendritic cell antigen processing and presentation